{
  "gene_name": "Synaptobrevin homolog YKT6",
  "term_label": "Golgi apparatus",
  "gene": "UniProtKB:O15498",
  "term_id": "GO:0005794",
  "gene_symbol": "YKT6"
}